{
  "gene": "UniProtKB:Q9Y2G5",
  "term_label": "peptide-O-fucosyltransferase activity",
  "gene_symbol": "POFUT2",
  "term_id": "GO:0046922",
  "gene_name": "GDP-fucose protein O-fucosyltransferase 2"
}